DNA secondary structure binding [GO:0000217] (molecular function) Sources: GOC:krc Subtypes: four-way junction DNA binding [GO:0000400], Y-form DNA binding [GO:0000403], heteroduplex DNA loop binding [GO:0000404], bubble DNA binding [GO:0000405], double-strand/single-strand DNA junction binding [GO:0000406], GO:0003680, DNA hairpin binding [GO:0032448], D-loop DNA binding [GO:0062037] Definition: Binding to a DNA secondary structure element such as a four-way junction, a bubble, a loop, Y-form DNA, or a double-strand/single-strand junction. Relationships: is_a DNA binding [GO:0003677]